{
  "term_id": "UNKNOWN:0003",
  "gene_name": "PC-esterase domain-containing protein 1A",
  "gene_symbol": "PCED1A",
  "term_label": "Unknown cellular component",
  "gene": "UniProtKB:Q9H1Q7"
}